{
  "gene_name": "N-acetyllactosaminide beta-1,3-N-acetylglucosaminyltransferase 4",
  "term_id": "GO:0008532",
  "gene": "UniProtKB:Q9C0J1",
  "term_label": "N-acetyllactosaminide beta-1,3-N-acetylglucosaminyltransferase activity",
  "gene_symbol": "B3GNT4"
}